{
  "term_label": "Unknown biological process",
  "gene": "UniProtKB:Q6ZU67",
  "term_id": "UNKNOWN:0002",
  "gene_symbol": "BEND4",
  "gene_name": "BEN domain-containing protein 4"
}